{
  "term_id": "GO:0043039",
  "gene_symbol": "YARS2",
  "gene": "UniProtKB:Q9Y2Z4",
  "gene_name": "Tyrosine--tRNA ligase, mitochondrial",
  "term_label": "tRNA aminoacylation"
}